ethanolamine transmembrane transporter activity [GO:0034228] (MF) References: PMID:3514579 Sources: GOC:rn Definition: Enables the transfer of ethanolamine from one side of a membrane to the other. Ethanolamine (2-aminoethanol, monoethanolamine) is an amino alcohol that occurs widely in living organisms as a constituent of certain types of phospholipids, such as phosphatidylethanolamine. Also known as: 2-aminoethanol transmembrane transporter activity, ethanolamine permease activity, monoethanolamine transmembrane transporter activity Relationships: is a type of amine transmembrane transporter activity [GO:0005275]; is a type of alcohol transmembrane transporter activity [GO:0015665]; is part of ethanolamine transport [GO:0034229]